{
  "term_id": "GO:0038100",
  "gene": "UniProtKB:P0CG36",
  "gene_name": "Cryptic family protein 1B",
  "term_label": "nodal binding",
  "gene_symbol": "CFC1B"
}